{
  "term_id": "GO:0097225",
  "gene_name": "Cilia- and flagella-associated protein 69",
  "term_label": "sperm midpiece",
  "gene": "UniProtKB:A5D8W1",
  "gene_symbol": "CFAP69"
}